positive regulation of border follicle cell delamination [GO:0030711] (biological process) Relationships: is a type of regulation of border follicle cell delamination [GO:0030710]; is a type of positive regulation of biological process [GO:0048518]; positively regulates GO:0030709 Definition: Any process that increases the frequency, rate or extent of border cell delamination. References: PMID:10822261 Also known as: positive regulation of border cell delamination, up regulation of border follicle cell delamination, up-regulation of border follicle cell delamination, upregulation of border follicle cell delamination, activation of border follicle cell delamination, stimulation of border follicle cell delamination